{
  "term_label": "positive regulation of cell differentiation",
  "gene": "UniProtKB:P11362",
  "gene_symbol": "FGFR1",
  "term_id": "GO:0045597",
  "gene_name": "Fibroblast growth factor receptor 1"
}